{
  "term_label": "Unknown cellular component",
  "gene_symbol": "LINC00696",
  "term_id": "UNKNOWN:0003",
  "gene_name": "Putative uncharacterized protein encoded by LINC00696",
  "gene": "UniProtKB:Q6ZRV3"
}